{
  "gene_name": "Angiotensin-converting enzyme 2",
  "term_id": "GO:0005615",
  "gene": "UniProtKB:Q9BYF1",
  "term_label": "extracellular space",
  "gene_symbol": "ACE2"
}